{
  "term_id": "GO:0007186",
  "term_label": "G protein-coupled receptor signaling pathway",
  "gene_symbol": "OR5D13",
  "gene_name": "Olfactory receptor 5D13",
  "gene": "UniProtKB:Q8NGL4"
}